right lung morphogenesis [GO:0060461] (biological process) Sources: GOC:dph, GOC:mtg_lung Definition: The process in which anatomical structures of the right lung are generated and organized. Relationships: is a type of lung morphogenesis [GO:0060425]; is part of GO:0060458